polysaccharide transmembrane transporter activity [GO:0015159] (molecular function) Sources: GOC:ai, GOC:mtg_transport, ISBN:0815340729 Relationships: is_a carbohydrate transmembrane transporter activity [GO:0015144]; is a type of macromolecule transmembrane transporter activity [GO:0022884]; is part of polysaccharide transport [GO:0015774] Subtypes: beta-glucan transmembrane transporter activity [GO:0015160], arabinan transmembrane transporter activity [GO:0042901], dextrin transmembrane transporter activity [GO:0042957] Definition: Enables the transfer of polysaccharides from one side of a membrane to the other. A polysaccharide is a polymer of many (typically more than 10) monosaccharide residues linked glycosidically.